cell migration involved in heart development [GO:0060973] (biological process) Definition: The orderly movement of a cell from one site to another that will contribute to the progression of the heart over time, from its initial formation, to the mature organ. Relationships: is_a GO:0016477; is part of GO:0007507 Sources: GOC:mtg_heart Subtypes: cardiac neural crest cell migration involved in outflow tract morphogenesis [GO:0003253], cell migration involved in endocardial cushion formation [GO:0003273], cell migration involved in heart jogging [GO:0003305], cell migration to the midline involved in heart development [GO:0003318], proepicardium cell migration involved in pericardium morphogenesis [GO:0003345], epicardium-derived cell migration to the myocardium [GO:0003346], cell migration involved in heart formation [GO:0060974], cell migration involved in coronary vasculogenesis [GO:0060980], cell migration involved in coronary angiogenesis [GO:0060981]